plant-type cell wall biogenesis [GO:0009832] (biological process) Also known as: cell wall anabolism, cell wall assembly, cell wall biosynthetic process, cell wall formation, cell wall synthesis, cellulose and pectin-containing cell wall biogenesis Subtypes: plant-type primary cell wall biogenesis [GO:0009833], plant-type secondary cell wall biogenesis [GO:0009834] Relationships: is a type of GO:0042546; is a type of plant-type cell wall organization or biogenesis [GO:0071669] Sources: GOC:go_curators, GOC:lr, GOC:mtg_sensu Definition: A cellular process that results in the biosynthesis of constituent macromolecules, assembly, and arrangement of constituent parts of a cellulose and pectin-containing cell wall. An example of this is found in Arabidopsis thaliana.